cholesterol import [GO:0070508] (biological process) Sources: GOC:BHF, GOC:rl Definition: The directed movement of cholesterol into a cell or organelle. Relationships: is a type of GO:0030301 Also known as: cholesterol uptake Regulation: regulated by regulation of cholesterol import [GO:0060620]; negatively regulated by negative regulation of cholesterol import [GO:0060621]; positively regulated by positive regulation of cholesterol import [GO:1904109]